{
  "gene_symbol": "GPATCH2",
  "gene_name": "G patch domain-containing protein 2",
  "term_label": "Unknown biological process",
  "gene": "UniProtKB:Q9NW75",
  "term_id": "UNKNOWN:0002"
}